{
  "gene": "UniProtKB:Q9Y5W3",
  "gene_symbol": "KLF2",
  "term_label": "DNA-binding transcription factor activity, RNA polymerase II-specific",
  "gene_name": "Krueppel-like factor 2",
  "term_id": "GO:0000981"
}